regulation of protein localization to synapse [GO:1902473] (biological process) References: PMID:22588719 Sources: GOC:TermGenie, GOC:kmv Definition: Any process that modulates the frequency, rate or extent of protein localization to synapse. Relationships: is_a regulation of protein localization [GO:0032880]; regulates protein localization to synapse [GO:0035418] Subtypes: regulation of neurotransmitter receptor localization to postsynaptic specialization membrane [GO:0098696], regulation of neurotransmitter receptor transport, endosome to postsynaptic membrane [GO:0099152], GO:1902474, regulation of protein localization to presynapse [GO:1905384] Also known as: regulation of protein localisation to synapse